{
  "gene_symbol": "IFNA14",
  "gene": "UniProtKB:P01570",
  "gene_name": "Interferon alpha-14",
  "term_label": "response to exogenous dsRNA",
  "term_id": "GO:0043330"
}